{
  "term_id": "GO:0030864",
  "gene": "UniProtKB:Q8NFW9",
  "gene_symbol": "MYRIP",
  "term_label": "cortical actin cytoskeleton",
  "gene_name": "Rab effector MyRIP"
}